{
  "term_label": "mitochondrion",
  "gene_symbol": "COX7B",
  "gene_name": "Cytochrome c oxidase subunit 7B, mitochondrial",
  "gene": "UniProtKB:P24311",
  "term_id": "GO:0005739"
}